{
  "gene": "UniProtKB:Q96DC7",
  "term_label": "Unknown cellular component",
  "gene_name": "Transmembrane and coiled-coil domain-containing protein 6",
  "term_id": "UNKNOWN:0003",
  "gene_symbol": "TMCO6"
}